positive regulation of centriole-centriole cohesion [GO:1903127] (biological process) References: PMID:24554434 Sources: GOC:TermGenie, GOC:als, GO_REF:0000058 Definition: Any process that activates or increases the frequency, rate or extent of centriole-centriole cohesion. Relationships: is a type of GO:0030997; is a type of positive regulation of cell cycle process [GO:0090068]; positively regulates centriole-centriole cohesion [GO:0010457] Also known as: up regulation of centriole-centriole cohesion, up-regulation of centriole-centriole cohesion, upregulation of centriole-centriole cohesion, activation of centriole-centriole cohesion